photosynthesis [GO:0015979] (biological process) Definition: The synthesis by organisms of organic chemical compounds, especially carbohydrates, from carbon dioxide (CO2) using energy obtained from light rather than from the oxidation of chemical compounds. Regulation: RO_0002211 by regulation of photosynthesis [GO:0010109]; negatively regulated by negative regulation of photosynthesis [GO:1905156]; positively regulated by positive regulation of photosynthesis [GO:1905157] Relationships: is a type of metabolic process [GO:0008152] Sources: ISBN:0198547684